2-dehydropantoate aldolase activity [GO:0050013] (molecular function) Definition: Catalysis of the reaction: 2-dehydropantoate = 3-methyl-2-oxobutanoate + formaldehyde. Relationships: is a type of aldehyde-lyase activity [GO:0016832] Sources: EC:4.1.2.12, MetaCyc:KETOPANTOALDOLASE-RXN Also known as: ketopantoaldolase activity, 2-dehydropantoate formaldehyde-lyase (3-methyl-2-oxobutanoate-forming), 2-dehydropantoate formaldehyde-lyase activity